{
  "term_label": "basolateral plasma membrane",
  "gene": "UniProtKB:Q86UG4",
  "gene_symbol": "SLCO6A1",
  "gene_name": "Solute carrier organic anion transporter family member 6A1",
  "term_id": "GO:0016323"
}